myoblast fate commitment in trunk [GO:0014715] (BP) Relationships: is a type of myoblast fate commitment [GO:0048625] Definition: The process taking place in the trunk whereby the developmental fate of a cell becomes restricted such that it will develop into a myoblast. A myoblast is a mononucleate cell type that, by fusion with other myoblasts, gives rise to the myotubes that eventually develop into skeletal muscle fibers. Sources: CL:0000056, GOC:mtg_muscle